{
  "gene": "UniProtKB:Q3MJ40",
  "term_id": "UNKNOWN:0002",
  "gene_symbol": "CCDC144BP",
  "gene_name": "Putative coiled-coil domain-containing protein 144B",
  "term_label": "Unknown biological process"
}